{
  "term_label": "Unknown cellular component",
  "term_id": "UNKNOWN:0003",
  "gene_name": "Pro-interleukin-16",
  "gene_symbol": "IL16",
  "gene": "UniProtKB:Q14005"
}